regulation of vitamin D receptor signaling pathway [GO:0070562] (biological process) Definition: Any process that modulates the frequency, rate or extent of vitamin D receptor signaling pathway activity. Relationships: is a type of regulation of response to nutrient levels [GO:0032107]; is a type of regulation of intracellular signal transduction [GO:1902531]; regulates GO:0070561 Sources: GOC:BHF, GOC:mah Subtypes: negative regulation of vitamin D receptor signaling pathway [GO:0070563], positive regulation of vitamin D receptor signaling pathway [GO:0070564] Also known as: regulation of VDR signaling pathway, regulation of vitamin D receptor signalling pathway